{
  "gene_symbol": "SNX25",
  "term_label": "Unknown biological process",
  "gene": "UniProtKB:Q9H3E2",
  "term_id": "UNKNOWN:0002",
  "gene_name": "Sorting nexin-25"
}